regulation of cilium movement [GO:0003352] (biological process) Sources: GOC:dph Also known as: regulation of microtubule-based flagellum movement, regulation of flagellar movement, regulation of flagellum movement Note: Note that we deem cilium and microtubule-based flagellum to be equivalent. Subtypes: positive regulation of cilium movement [GO:0003353], negative regulation of cilium movement [GO:0003354], GO:0003356, regulation of cilium movement involved in cell motility [GO:0060295], maintenance of ciliary planar beating movement pattern [GO:0120221] Definition: Any process that modulates the rate, frequency, or extent of cilium movement, the directed, self-propelled movement of a cilium. Relationships: is a type of regulation of microtubule-based movement [GO:0060632]; regulates cilium movement [GO:0003341]